{
  "gene": "UniProtKB:Q9H841",
  "gene_name": "NIPA-like protein 2",
  "term_label": "Unknown molecular function",
  "term_id": "UNKNOWN:0001",
  "gene_symbol": "NIPAL2"
}